{
  "gene_name": "Leucine-rich repeat-containing protein 26",
  "term_label": "voltage-gated potassium channel complex",
  "term_id": "GO:0008076",
  "gene": "UniProtKB:Q2I0M4",
  "gene_symbol": "LRRC26"
}